{
  "term_id": "GO:0015630",
  "term_label": "microtubule cytoskeleton",
  "gene": "UniProtKB:Q8WWK9",
  "gene_symbol": "CKAP2",
  "gene_name": "Cytoskeleton-associated protein 2"
}